{
  "gene_name": "Endothelial transcription factor GATA-2",
  "gene_symbol": "GATA2",
  "term_id": "GO:0000978",
  "gene": "UniProtKB:P23769",
  "term_label": "RNA polymerase II cis-regulatory region sequence-specific DNA binding"
}